{
  "gene_symbol": "IGLV10-54",
  "gene": "UniProtKB:A0A075B6I4",
  "term_id": "GO:0006955",
  "gene_name": "Immunoglobulin lambda variable 10-54",
  "term_label": "immune response"
}